1-acylglycerophosphocholine O-acyltransferase activity [GO:0047184] (molecular function) Sources: EC:2.3.1.23, MetaCyc:2.3.1.23-RXN Definition: Catalysis of the reaction: 1-acyl-sn-glycero-3-phosphocholine + acyl-CoA = phosphatidylcholine + CoA. Relationships: is a type of O-acyltransferase activity [GO:0008374] Also known as: 1-acyl-sn-glycero-3-phosphocholine acyltransferase activity, acyl coenzyme A-monoacylphosphatidylcholine acyltransferase activity, acyl-CoA:1-acyl-glycero-3-phosphocholine transacylase activity, acyl-CoA:1-acyl-sn-glycero-3-phosphocholine O-acyltransferase activity, lysolecithin acyltransferase activity, lysophosphatide acyltransferase activity, lysophosphatidylcholine acyltransferase activity